{
  "gene": "UniProtKB:Q9NUD5",
  "gene_symbol": "ZCCHC3",
  "term_id": "GO:0071360",
  "term_label": "cellular response to exogenous dsRNA",
  "gene_name": "Zinc finger CCHC domain-containing protein 3"
}